toll-like receptor 9 signaling pathway [GO:0034162] (biological process) Definition: The series of molecular signals initiated by a ligand binding to the endolysosomal toll-like receptor 9. Regulation: regulated by GO:0034163; negatively regulated by negative regulation of toll-like receptor 9 signaling pathway [GO:0034164]; positively regulated by GO:0034165 Relationships: is a type of endolysosomal toll-like receptor signaling pathway [GO:0140894] References: PMID:16551253, PMID:17328678 Sources: GOC:add Also known as: TLR9 signaling pathway, toll-like receptor 9 signalling pathway